{
  "gene_symbol": "FAM209B",
  "term_label": "Unknown molecular function",
  "gene_name": "Protein FAM209B",
  "gene": "UniProtKB:Q5JX69",
  "term_id": "UNKNOWN:0001"
}